{
  "gene_name": "Semaphorin-4B",
  "term_id": "GO:0007411",
  "gene_symbol": "SEMA4B",
  "term_label": "axon guidance",
  "gene": "UniProtKB:Q9NPR2"
}